{
  "term_id": "GO:0060271",
  "gene_symbol": "TTC39C",
  "gene": "UniProtKB:Q8N584",
  "gene_name": "Tetratricopeptide repeat protein 39C",
  "term_label": "cilium assembly"
}